{
  "term_label": "lysosomal membrane",
  "gene_symbol": "LAPTM4A",
  "gene_name": "Lysosomal-associated transmembrane protein 4A",
  "term_id": "GO:0005765",
  "gene": "UniProtKB:Q15012"
}